{
  "term_label": "keratin filament",
  "gene_symbol": "KRT27",
  "term_id": "GO:0045095",
  "gene_name": "Keratin, type I cytoskeletal 27",
  "gene": "UniProtKB:Q7Z3Y8"
}